{
  "gene_symbol": "CFLAR",
  "term_id": "GO:0004197",
  "gene": "UniProtKB:O15519",
  "gene_name": "CASP8 and FADD-like apoptosis regulator",
  "term_label": "cysteine-type endopeptidase activity"
}